{
  "gene": "UniProtKB:O00299",
  "gene_name": "Chloride intracellular channel protein 1",
  "gene_symbol": "CLIC1",
  "term_id": "GO:0006821",
  "term_label": "chloride transport"
}